{
  "gene": "UniProtKB:Q9UQR0",
  "term_label": "negative regulation of DNA-templated transcription",
  "gene_symbol": "SCML2",
  "term_id": "GO:0045892",
  "gene_name": "Sex comb on midleg-like protein 2"
}